{
  "term_id": "GO:0007165",
  "gene_symbol": "MAGI3",
  "gene_name": "Membrane-associated guanylate kinase, WW and PDZ domain-containing protein 3",
  "term_label": "signal transduction",
  "gene": "UniProtKB:Q5TCQ9"
}